{
  "term_label": "positive regulation of transcription by RNA polymerase II",
  "gene": "UniProtKB:Q7Z6R9",
  "gene_name": "Transcription factor AP-2-delta",
  "term_id": "GO:0045944",
  "gene_symbol": "TFAP2D"
}